{
  "gene_name": "Small ribosomal subunit protein uS17",
  "term_label": "cytosolic small ribosomal subunit",
  "term_id": "GO:0022627",
  "gene_symbol": "RPS11",
  "gene": "UniProtKB:P62280"
}